{
  "term_label": "neuron projection development",
  "gene_name": "Receptor-type tyrosine-protein phosphatase kappa",
  "term_id": "GO:0031175",
  "gene": "UniProtKB:Q15262",
  "gene_symbol": "PTPRK"
}